{
  "gene": "UniProtKB:P20132",
  "gene_name": "L-serine dehydratase_L-threonine deaminase",
  "gene_symbol": "SDS",
  "term_id": "GO:0006567",
  "term_label": "L-threonine catabolic process"
}